{
  "gene_name": "Structural maintenance of chromosomes protein 1B",
  "gene": "UniProtKB:Q8NDV3",
  "term_label": "DNA binding",
  "gene_symbol": "SMC1B",
  "term_id": "GO:0003677"
}